{
  "term_label": "intracellular signal transduction",
  "gene_name": "Tyrosine-protein kinase JAK2",
  "gene": "UniProtKB:O60674",
  "gene_symbol": "JAK2",
  "term_id": "GO:0035556"
}